{
  "gene": "UniProtKB:P08708",
  "gene_symbol": "RPS17",
  "term_id": "UNKNOWN:0002",
  "term_label": "Unknown biological process",
  "gene_name": "Small ribosomal subunit protein eS17"
}